{
  "term_id": "GO:0016020",
  "term_label": "membrane",
  "gene": "UniProtKB:Q8WY21",
  "gene_symbol": "SORCS1",
  "gene_name": "VPS10 domain-containing receptor SorCS1"
}